taxane 13-alpha-hydroxylase activity [GO:0050598] (molecular function) Also known as: taxane 13a-hydroxylase activity, taxa-4(20),11-dien-5alpha-ol,NADPH:oxygen oxidoreductase (13alpha-hydroxylating), taxane 13alpha-hydroxylase activity Definition: Catalysis of the reaction: H+ + NADPH + O2 + taxa-4(20),11-dien-5alpha-ol = H2O + NADP+ + taxa-4(20),11-dien-5alpha,13alpha-diol. Relationships: is a type of oxidoreductase activity, acting on paired donors, with incorporation or reduction of molecular oxygen, NAD(P)H as one donor, and incorporation of one atom of oxygen [GO:0016709] Sources: EC:1.14.14.106, RHEA:18949